Meynert cell differentiation [GO:1905270] (biological process) Definition: The process in which a relatively unspecialized cell acquires the specialized features of a Meynert cell. Relationships: is a type of pyramidal neuron differentiation [GO:0021859]; is a type of cerebral cortex neuron differentiation [GO:0021895] References: PMID:4142639 Sources: GOC:TermGenie, GO_REF:0000086